{
  "gene_symbol": "TMEM275",
  "term_label": "Unknown molecular function",
  "gene_name": "Transmembrane protein 275",
  "term_id": "UNKNOWN:0001",
  "gene": "UniProtKB:A0A0U1RQS6"
}